positive regulation of toll-like receptor 9 signaling pathway [GO:0034165] (biological process) References: PMID:16551253, PMID:17328678 Sources: GOC:add Subtypes: positive regulation of toll-like receptor 9 signaling pathway by B cell receptor internalization [GO:1901245] Definition: Any process that activates or increases the frequency, rate, or extent of toll-like receptor 9 signaling pathway. Relationships: is a type of regulation of toll-like receptor 9 signaling pathway [GO:0034163]; is a type of positive regulation of pattern recognition receptor signaling pathway [GO:0062208]; is a type of positive regulation of intracellular signal transduction [GO:1902533]; positively regulates toll-like receptor 9 signaling pathway [GO:0034162] Also known as: positive regulation of TLR9 signaling pathway, positive regulation of toll-like receptor 9 signalling pathway